{
  "gene_symbol": "AIRE",
  "gene_name": "Autoimmune regulator",
  "term_id": "GO:0002509",
  "gene": "UniProtKB:O43918",
  "term_label": "central tolerance induction to self antigen"
}